positive regulation of glutamate secretion, neurotransmission [GO:1903296] (biological process) Definition: Any process that activates or increases the frequency, rate or extent of glutamate secretion, where glutamate acts as a neurotransmitter. Subtypes: positive regulation of glutamate neurotransmitter secretion in response to membrane depolarization [GO:0061646] Also known as: up regulation of glutamate secretion, neurotransmission, up-regulation of glutamate secretion, neurotransmission, upregulation of glutamate secretion, neurotransmission, activation of glutamate secretion, neurotransmission Note: An example of this is Rab3gap1 in mouse (Q80UJ7) in PMID:16782817 inferred from mutant phenotype Relationships: is a type of GO:0001956; is a type of positive regulation of glutamate secretion [GO:0014049]; is a type of GO:0051968; is a type of regulation of glutamate secretion, neurotransmission [GO:1903294]; positively regulates glutamate secretion, neurotransmission [GO:0061535] References: PMID:16782817 Sources: GOC:TermGenie, GO_REF:0000058